{
  "gene_symbol": "TRARG1",
  "term_label": "endosome to plasma membrane protein transport",
  "term_id": "GO:0099638",
  "gene": "UniProtKB:Q8IXB3",
  "gene_name": "Trafficking regulator of GLUT4 1"
}